{
  "gene_name": "Cadherin-1",
  "term_id": "GO:0016342",
  "term_label": "catenin complex",
  "gene": "UniProtKB:P12830",
  "gene_symbol": "CDH1"
}